{
  "term_id": "UNKNOWN:0002",
  "gene_name": "PRO2179",
  "gene_symbol": "Q9H3A6",
  "term_label": "Unknown biological process",
  "gene": "UniProtKB:Q9H3A6"
}